regulation of macrophage apoptotic process [GO:2000109] (biological process) Definition: Any process that modulates the frequency, rate or extent of macrophage apoptotic process. Relationships: is a type of regulation of myeloid cell apoptotic process [GO:0033032]; is a type of regulation of leukocyte apoptotic process [GO:2000106]; regulates macrophage apoptotic process [GO:0071888] Sources: GOC:BHF, GOC:mtg_apoptosis Also known as: regulation of macrophage apoptosis, regulation of AICD, regulation of activation-induced cell death Subtypes: negative regulation of macrophage apoptotic process [GO:2000110], GO:2000111